{
  "gene_name": "Peroxisomal biogenesis factor 3",
  "term_label": "protein-macromolecule adaptor activity",
  "gene_symbol": "PEX3",
  "term_id": "GO:0030674",
  "gene": "UniProtKB:P56589"
}